symbiont-mediated suppression of host neurotransmitter secretion [GO:0044762] (biological process) Relationships: is a type of symbiont-mediated perturbation of host neurotransmitter secretion [GO:0044079] Definition: A process in which a symbiont inhibits or disrupts the regulated release of a neurotransmitter from a cell in its host organism. References: PMID:1328520, PMID:7901002 Also known as: negative regulation by symbiont of host neurotransmitter secretion